accessory nerve maturation [GO:0021606] (biological process) Also known as: CN XI maturation, spinal accessory nerve maturation Sources: GOC:cls, GOC:dgh, GOC:dph, GOC:jid, GO_REF:0000021 Relationships: is a type of GO:0021605; is part of GO:0021565 Definition: A developmental process, independent of morphogenetic (shape) change, that is required for the accessory nerve to attain its fully functional state. The spinal branch of this motor nerve innervates the trapezius and the sternocleidomastoid muscles. The cranial branch joins the vagus nerve and innervates the same targets as the vagus nerve.